{
  "term_label": "plasma membrane",
  "gene": "UniProtKB:A0A0K2S4Q6",
  "gene_symbol": "CD300H",
  "term_id": "GO:0005886",
  "gene_name": "Protein CD300H"
}